{
  "term_id": "GO:0030154",
  "term_label": "cell differentiation",
  "gene": "UniProtKB:Q13133",
  "gene_symbol": "NR1H3",
  "gene_name": "Oxysterols receptor LXR-alpha"
}